{
  "gene_name": "Rhomboid-related protein 4",
  "gene_symbol": "RHBDD1",
  "term_id": "GO:0034620",
  "gene": "UniProtKB:Q8TEB9",
  "term_label": "cellular response to unfolded protein"
}